{
  "gene_name": "AMSH-like protease",
  "term_id": "GO:0016020",
  "gene": "UniProtKB:Q96FJ0",
  "term_label": "membrane",
  "gene_symbol": "STAMBPL1"
}